{
  "gene": "UniProtKB:Q2TB18",
  "term_id": "UNKNOWN:0002",
  "gene_name": "Protein asteroid homolog 1",
  "gene_symbol": "ASTE1",
  "term_label": "Unknown biological process"
}